alphaM-beta2 integrin-CD63 complex [GO:0070558] (cellular component) Definition: A protein complex that consists of an alphaM-beta2 integrin complex bound to membrane protein CD63, a member of the tetraspan family. Relationships: is a type of GO:0098797 References: PMID:8871662 Also known as: ITGAM-ITGB2-CD63 complex